{
  "term_label": "detection of chemical stimulus involved in sensory perception of smell",
  "gene_symbol": "OR2T33",
  "gene_name": "Olfactory receptor 2T33",
  "term_id": "GO:0050911",
  "gene": "UniProtKB:Q8NG76"
}